convergent extension involved in neural plate elongation [GO:0022007] (biological process) Regulation: RO_0002211 by regulation of convergent extension involved in neural plate elongation [GO:1904130]; negatively regulated by negative regulation of convergent extension involved in neural plate elongation [GO:1904131]; positively regulated by GO:1904132 References: PMID:13679871, PMID:15806586 Sources: GOC:cls, GOC:dgh, GOC:dph, GOC:jid, GO_REF:0000021 Definition: The process of directed cell movement in the neural plate resulting in tissue elongation via intercalation of adjacent cells in an epithelial sheet at the midline, leading to narrowing and lengthening of the neural plate. Relationships: is a type of GO:0060027; is a type of convergent extension involved in organogenesis [GO:0060029]; is part of GO:0014022